{
  "gene": "UniProtKB:P61073",
  "term_label": "immune response",
  "gene_name": "C-X-C chemokine receptor type 4",
  "gene_symbol": "CXCR4",
  "term_id": "GO:0006955"
}